translational attenuation [GO:0009386] (biological process) Relationships: is a type of regulation of translation [GO:0006417] References: PMID:15694341, PMID:15805513 Definition: Translational attenuation is a regulatory mechanism analogous to ribosome-mediated transcriptional attenuation. The system requires the presence of a short ORF, called a leader peptide, encoded in the mRNA upstream of the ribosome-binding site and start codon of the gene whose translation is to be regulated. Certain conditions, such as presence of the antibiotic tetracycline in bacteria or amino acid starvation, may cause slowing or stalling of the ribosome translating the leader peptide. The stalled ribosome masks a region of the mRNA and affects which of two alternative mRNA folded structures will form, therefore controlling whether or not a ribosome will bind and initiate translation of the downstream gene. Translational attenuation is analogous to ribosome-mediated transcriptional attenuation, in which mRNA remodeling caused by ribosome stalling regulates transcriptional termination rather than translational initiation.